notochord cell development [GO:0060035] (biological process) Definition: The process whose specific outcome is the progression of a notochord cell over time, from its formation to its mature structure. Cell development does not include the steps involved in committing a cell to a specific fate. Relationships: is a type of cell development [GO:0048468]; is part of notochord cell differentiation [GO:0060034] Sources: GOC:dph